{
  "gene_symbol": "CLOCK",
  "term_label": "CLOCK-BMAL transcription complex",
  "gene": "UniProtKB:O15516",
  "term_id": "GO:1990513",
  "gene_name": "Circadian locomoter output cycles protein kaput"
}